{
  "term_id": "GO:0002286",
  "gene_name": "Interferon alpha-21",
  "gene": "UniProtKB:P01568",
  "term_label": "T cell activation involved in immune response",
  "gene_symbol": "IFNA21"
}